{
  "gene_name": "Profilin-3",
  "term_label": "positive regulation of actin filament bundle assembly",
  "term_id": "GO:0032233",
  "gene_symbol": "PFN3",
  "gene": "UniProtKB:P60673"
}